endo-1,4-beta-xylanase activity [GO:0031176] (MF) Sources: EC:3.2.1.8 Relationships: is a type of xylanase activity [GO:0097599] Definition: Catalysis of the endohydrolysis of (1->4)-beta-D-xylosidic linkages in xylans. Also known as: xylanase, 1,4-beta-D-xylan xylanohydrolase activity, 1,4-beta-xylan xylanohydrolase activity, beta-1,4-xylan xylanohydrolase activity, beta-1,4-xylanase activity, beta-D-xylanase activity, beta-xylanase activity, endo-(1,4)-beta-xylanase(1,4)-beta-xylan 4-xylanohydrolase activity, endo-(1->4)-beta-xylanase(1->4)-beta-xylan 4-xylanohydrolase activity, endo-1,4-beta-D-xylanase activity, endo-1,4-xylanase activity, endo-beta-1,4-xylanase activity